GTPase motor activity [GO:0061791] (molecular function) References: PMID:11242086 Sources: GOC:dph, GOC:vw Subtypes: ribosome translocase activity [GO:0180054], membrane scission GTPase motor activity [GO:1990606] Relationships: is_a cytoskeletal motor activity [GO:0003774]; is a type of GTPase activity [GO:0003924] Definition: A motor activity driven by GTP hydrolysis.